{
  "gene": "UniProtKB:Q8NGL0",
  "gene_symbol": "OR5L2",
  "term_id": "UNKNOWN:0003",
  "gene_name": "Olfactory receptor 5L2",
  "term_label": "Unknown cellular component"
}